conversion of methionyl-tRNA to N-formyl-methionyl-tRNA [GO:0071951] (biological process) References: PMID:5337045 Sources: GOC:jsg Definition: The modification process that results in the conversion of methionine charged on a tRNA(fMet) to N-formyl-methionine-tRNA(fMet). Relationships: is a type of charged-tRNA amino acid modification [GO:0019988]